{
  "gene_name": "5-hydroxytryptamine receptor 7",
  "term_label": "neurotransmitter receptor activity",
  "gene_symbol": "HTR7",
  "term_id": "GO:0030594",
  "gene": "UniProtKB:P34969"
}